{
  "term_label": "monoacylglycerol catabolic process",
  "gene": "UniProtKB:O95870",
  "term_id": "GO:0052651",
  "gene_name": "Phosphatidylserine lipase ABHD16A",
  "gene_symbol": "ABHD16A"
}